negative regulation of endoribonuclease activity [GO:0060702] (biological process) Relationships: is a type of negative regulation of catalytic activity [GO:0043086]; is a type of regulation of endoribonuclease activity [GO:0060699]; negatively regulates RNA endonuclease activity [GO:0004521] Definition: Any process that decreases the rate, frequency or extent of the catalysis of the hydrolysis of ester linkages within ribonucleic acid by creating internal breaks. Sources: GOC:dph, GOC:tb